{
  "gene": "UniProtKB:Q9GZR1",
  "gene_name": "Sentrin-specific protease 6",
  "term_id": "GO:0090169",
  "gene_symbol": "SENP6",
  "term_label": "regulation of spindle assembly"
}